phosphoglycerate kinase activity [GO:0004618] (molecular function) Sources: EC:2.7.2.3, RHEA:14801 Definition: Catalysis of the reaction: 3-phospho-D-glycerate + ATP = 3-phospho-D-glyceroyl phosphate + ADP + H+. Also known as: 3-PGK, 3-phosphoglycerate kinase activity, 3-phosphoglycerate phosphokinase activity, 3-phosphoglyceric acid kinase activity, 3-phosphoglyceric acid phosphokinase activity, 3-phosphoglyceric kinase activity, ATP-3-phospho-D-glycerate-1-phosphotransferase activity, ATP:3-phospho-D-glycerate 1-phosphotransferase activity, ATP:D-3-phosphoglycerate 1-phosphotransferase activity, PGK, glycerate 3-phosphate kinase activity, glycerophosphate kinase activity, phosphoglyceric acid kinase activity, phosphoglyceric kinase activity, phosphoglycerokinase activity Relationships: is a type of kinase activity [GO:0016301]; is a type of phosphotransferase activity, carboxyl group as acceptor [GO:0016774]